{
  "term_id": "UNKNOWN:0001",
  "gene_symbol": "WDR53",
  "gene_name": "WD repeat-containing protein 53",
  "gene": "UniProtKB:Q7Z5U6",
  "term_label": "Unknown molecular function"
}